{
  "term_id": "GO:0006312",
  "gene_symbol": "MSH3",
  "gene_name": "DNA mismatch repair protein Msh3",
  "gene": "UniProtKB:P20585",
  "term_label": "mitotic recombination"
}